presynapse assembly [GO:0099054] (biological process) Definition: The aggregation, arrangement and bonding together of a set of components to form a presynapse. Regulation: regulated by regulation of presynapse assembly [GO:1905606]; RO_0002212 by negative regulation of presynapse assembly [GO:1905607]; RO_0002213 by positive regulation of presynapse assembly [GO:1905608] Relationships: is a type of GO:0022607; is_a presynapse organization [GO:0099172]; is part of GO:0007416 Also known as: presynapse biogenesis, presynaptic terminal assembly References: PMID:24449494 Sources: GOC:PARL, GOC:bf, GOC:dos